{
  "gene_symbol": "ZNF565",
  "term_id": "GO:0005634",
  "gene": "UniProtKB:Q8N9K5",
  "term_label": "nucleus",
  "gene_name": "Zinc finger protein 565"
}